{
  "term_id": "UNKNOWN:0003",
  "gene_name": "Retinal dehydrogenase 2",
  "term_label": "Unknown cellular component",
  "gene": "UniProtKB:O94788",
  "gene_symbol": "ALDH1A2"
}